{
  "gene_name": "Heat shock protein beta-8",
  "gene": "UniProtKB:Q9UJY1",
  "gene_symbol": "HSPB8",
  "term_label": "cytoplasm",
  "term_id": "GO:0005737"
}